alphav-beta5 integrin-vitronectin complex [GO:0034997] (cellular component) Relationships: is a type of plasma membrane protein complex [GO:0098797] Also known as: ITGAV-ITGB5-VTN complex Definition: A protein complex that comprises one integrin alphav subunit, one integrin beta5 subunit, and vitronectin. References: PMID:1694173